{
  "term_label": "Unknown biological process",
  "gene": "UniProtKB:Q6ZS49",
  "gene_name": "Putative uncharacterized protein FLJ45831",
  "gene_symbol": "Q6ZS49",
  "term_id": "UNKNOWN:0002"
}